{
  "term_id": "GO:0006127",
  "gene": "UniProtKB:P43304",
  "gene_name": "Glycerol-3-phosphate dehydrogenase, mitochondrial",
  "term_label": "glycerol-3-phosphate shuttle",
  "gene_symbol": "GPD2"
}